{
  "gene": "UniProtKB:Q07075",
  "term_label": "extracellular space",
  "gene_name": "Glutamyl aminopeptidase",
  "term_id": "GO:0005615",
  "gene_symbol": "ENPEP"
}